{
  "term_label": "Unknown biological process",
  "gene_name": "Atrial natriuretic peptide-converting enzyme",
  "gene": "UniProtKB:Q9Y5Q5",
  "gene_symbol": "CORIN",
  "term_id": "UNKNOWN:0002"
}